{
  "gene_name": "IgG receptor FcRn large subunit p51",
  "term_label": "extracellular space",
  "gene": "UniProtKB:P55899",
  "term_id": "GO:0005615",
  "gene_symbol": "FCGRT"
}